postsynaptic endosome membrane [GO:0098895] (cellular component) Definition: The lipid bilayer surrounding a postsynaptic endosome. Relationships: is a type of endosome membrane [GO:0010008]; is part of postsynaptic endosome [GO:0098845] Sources: GOC:pz Subtypes: postsynaptic early endosome membrane [GO:0098896], postsynaptic recycling endosome membrane [GO:0098944]